{
  "gene_name": "Polycystin-2-like protein 1",
  "gene_symbol": "PKD2L1",
  "term_label": "detection of mechanical stimulus",
  "gene": "UniProtKB:Q9P0L9",
  "term_id": "GO:0050982"
}